succinyl-CoA catabolic process [GO:1901289] (biological process) Definition: The chemical reactions and pathways resulting in the breakdown of succinyl-CoA. Sources: GOC:TermGenie, GOC:yaf, UniPathway:UPA00929 Also known as: succinyl-CoA breakdown, succinyl-CoA catabolism, succinyl-CoA degradation Relationships: is a type of succinyl-CoA metabolic process [GO:0006104]; is a type of sulfur compound catabolic process [GO:0044273]; is a type of purine-containing compound catabolic process [GO:0072523]; is a type of GO:1901292